symbiont-mediated suppression of host JAK-STAT cascade via inhibition of host IRF9 activity [GO:0039560] (biological process) Note: This term is for annotation of symbiont proteins that counteract the host innate immune response. Also known as: disruption by virus of host JAK-STAT cascade via inhibition of host IRF9 activity, inhibition of host IRF9 by virus, inhibition of host interferon regulatory factor-9 by virus, suppression by virus of host IRF9 activity, suppression by virus of host JAK-STAT cascade via inhibition of host IRF9 activity, suppression by virus of host interferon regulatory factor 9 activity Definition: A process in which a symbiont interferes with, inhibits or disrupt a JAK-STAT signal cascade in the host organism by reducing the activity of host IRF9 (interferon regulatory factor-9), a transcription factor involved in the innate immune response. For example, viral infection triggers binding of IRF9 to phosphorylated STAT1 and STAT2, forming the ISGF3 complex. The ISGF3 complex migrates to the nucleus and activates transcription of IFN-responsive genes. Relationships: is a type of symbiont-mediated suppression of host JAK-STAT cascade [GO:0039514]; is a type of symbiont-mediated suppression of host innate immune response [GO:0052170] References: PMID:10388655, PMID:19109390